secondary neural tube formation [GO:0014021] (biological process) References: PMID:15327780 Sources: GOC:ef, ISBN:0878932585 Also known as: medullary cord biosynthesis, medullary cord formation, secondary neurulation, medullary rod cavitation, neural rod formation, secondary neural tube rod cavitation Relationships: is a type of embryonic epithelial tube formation [GO:0001838]; is part of neural tube formation [GO:0001841] Definition: The formation of the neural tube by coalescence of mesenchymal cells followed by their conversion to epithelial cells to form a solid cord that subsequently hollows out (cavitates) to create a hollow tube. Secondary neurulation is the typical mechanism of formation of the neural tube posterior to the posterior neuropore in mammals.